{
  "gene_symbol": "CCL8",
  "gene_name": "C-C motif chemokine 8",
  "term_label": "chemokine-mediated signaling pathway",
  "term_id": "GO:0070098",
  "gene": "UniProtKB:P80075"
}